response to rest involved in regulation of muscle adaptation [GO:0014893] (biological process) Definition: Any process that results in a change in state or activity of a cell or an organism (in terms of movement, secretion, enzyme production, gene expression, etc.) as a result of a rest stimulus. This process occurs as part of the regulation of muscle adaptation. Sources: GOC:mtg_muscle Relationships: is_a response to muscle inactivity involved in regulation of muscle adaptation [GO:0014877]